double-stranded telomeric DNA binding [GO:0003691] (molecular function) Sources: GOC:jl, ISBN:0321000382 Definition: Binding to double-stranded telomere-associated DNA. Relationships: is_a GO:0003690; is a type of telomeric DNA binding [GO:0042162]